{
  "gene_symbol": "FDXACB1",
  "gene_name": "Ferredoxin-fold anticodon-binding domain-containing protein 1",
  "term_id": "GO:0070042",
  "term_label": "rRNA (uridine-N3-)-methyltransferase activity",
  "gene": "UniProtKB:Q9BRP7"
}